{
  "term_label": "Unknown biological process",
  "term_id": "UNKNOWN:0002",
  "gene_symbol": "ZNF593",
  "gene": "UniProtKB:O00488",
  "gene_name": "Zinc finger protein 593"
}